{
  "gene_name": "Spermidine_spermine N(1)-acetyltransferase-like protein 1",
  "gene": "UniProtKB:Q86VE3",
  "term_label": "diamine N-acetyltransferase activity",
  "term_id": "GO:0004145",
  "gene_symbol": "SATL1"
}